{
  "term_id": "GO:0004115",
  "gene": "UniProtKB:O76083",
  "gene_name": "High affinity cGMP-specific 3',5'-cyclic phosphodiesterase 9A",
  "gene_symbol": "PDE9A",
  "term_label": "3',5'-cyclic-AMP phosphodiesterase activity"
}